{
  "gene": "UniProtKB:Q9NPC6",
  "term_id": "GO:0003779",
  "gene_symbol": "MYOZ2",
  "term_label": "actin binding",
  "gene_name": "Myozenin-2"
}